laminaritriose transport [GO:2001097] (biological process) Definition: The directed movement of a laminaritrioseacetate into, out of or within a cell, or between cells, by means of some agent such as a transporter or pore. Sources: GOC:mengo_curators Relationships: is a type of trisaccharide transport [GO:2001088] Regulation: regulated by regulation of laminaritriose transport [GO:1900303]; negatively regulated by negative regulation of laminaritriose transport [GO:1900304]; positively regulated by GO:1900305